mRNA branch site recognition [GO:0000348] (BP) Definition: Recognition of the pre-mRNA branch site sequence by components of the assembling spliceosome. Relationships: is a type of protein-RNA complex assembly [GO:0022618]; is part of spliceosomal complex assembly [GO:0000245] Also known as: nuclear mRNA branch site recognition, U12-type nuclear mRNA branch site recognition, U2-type nuclear mRNA branch site recognition, spliceosomal A complex biosynthesis, spliceosomal A complex formation, spliceosomal B complex biosynthesis, spliceosomal B complex formation Note: Note that this step represents the formation of the B complex (yeast) or the A complex (mammalian). Sources: GOC:krc, ISBN:0879695897